{
  "gene": "UniProtKB:A0A0A0MT99",
  "gene_name": "Immunoglobulin lambda joining 3 (Fragment)",
  "gene_symbol": "IGLJ3",
  "term_label": "Unknown molecular function",
  "term_id": "UNKNOWN:0001"
}